{
  "gene": "UniProtKB:P48730",
  "gene_name": "Casein kinase I isoform delta",
  "term_label": "nucleus",
  "gene_symbol": "CSNK1D",
  "term_id": "GO:0005634"
}